{
  "gene_name": "Protein Wnt-5b",
  "term_label": "canonical Wnt signaling pathway",
  "gene_symbol": "WNT5B",
  "gene": "UniProtKB:Q9H1J7",
  "term_id": "GO:0060070"
}